regulation of peptidyl-lysine acetylation [GO:2000756] (biological process) Sources: GOC:obol Definition: Any process that modulates the frequency, rate or extent of peptidyl-lysine acetylation. Subtypes: negative regulation of peptidyl-lysine acetylation [GO:2000757], positive regulation of peptidyl-lysine acetylation [GO:2000758], regulation of N-terminal peptidyl-lysine acetylation [GO:2000759] Relationships: is a type of GO:1901983; regulates peptidyl-lysine acetylation [GO:0018394]